{
  "gene": "UniProtKB:A0A0B4J266",
  "gene_symbol": "TRAV41",
  "term_label": "Unknown cellular component",
  "term_id": "UNKNOWN:0003",
  "gene_name": "T cell receptor alpha variable 41"
}